{
  "gene_symbol": "MAD2L2",
  "gene_name": "Mitotic spindle assembly checkpoint protein MAD2B",
  "term_id": "UNKNOWN:0001",
  "term_label": "Unknown molecular function",
  "gene": "UniProtKB:Q9UI95"
}